{
  "gene_symbol": "CSNK1G1",
  "gene_name": "Casein kinase I isoform gamma-1",
  "term_label": "endocytosis",
  "term_id": "GO:0006897",
  "gene": "UniProtKB:Q9HCP0"
}